inferior olivary nucleus morphogenesis [GO:0021714] (biological process) Also known as: inferior olive morphogenesis Sources: GOC:cls, GOC:dgh, GOC:dph, GOC:jid, GO_REF:0000021 Relationships: is a type of anatomical structure morphogenesis [GO:0009653]; is part of GO:0021579; BFO_0000050 inferior olivary nucleus development [GO:0021713] Definition: The process in which the anatomical structure of the inferior olivary nucleus is generated and organized. The inferior olivary nucleus is a capsule-shaped structure in the ventral medulla located just lateral and dorsal to the medullary pyramids. Neurons in the inferior olivary nucleus are the source of climbing fiber input to the cerebellar cortex; these neurons have been implicated in various functions, such as learning and timing of movements.